{
  "gene": "UniProtKB:Q9UPU5",
  "gene_name": "Ubiquitin carboxyl-terminal hydrolase 24",
  "term_label": "cytosol",
  "term_id": "GO:0005829",
  "gene_symbol": "USP24"
}